{
  "gene": "UniProtKB:Q9NRZ5",
  "gene_name": "1-acyl-sn-glycerol-3-phosphate acyltransferase delta",
  "term_id": "GO:0005741",
  "gene_symbol": "AGPAT4",
  "term_label": "mitochondrial outer membrane"
}